{
  "gene_name": "Zinc finger and BTB domain-containing protein 7C",
  "term_label": "DNA-binding transcription factor activity, RNA polymerase II-specific",
  "gene": "UniProtKB:A1YPR0",
  "gene_symbol": "ZBTB7C",
  "term_id": "GO:0000981"
}